thylakoid [GO:0009579] (cellular component) Also known as: photosynthetic membrane Subtypes: bacterial thylakoid [GO:0030075], plastid thylakoid [GO:0031976], GO:0070116 Note: A thylakoid is not considered an organelle, but some thylakoids are part of organelles. Definition: A membranous cellular structure that bears the photosynthetic pigments in plants, algae, and cyanobacteria. In cyanobacteria thylakoids are of various shapes and are attached to, or continuous with, the plasma membrane. In eukaryotes they are flattened, membrane-bounded disk-like structures located in the chloroplasts; in the chloroplasts of higher plants the thylakoids form dense stacks called grana. Isolated thylakoid preparations can carry out photosynthetic electron transport and the associated phosphorylation. Relationships: is a type of GO:0043232 Sources: GOC:ds, GOC:mtg_sensu, ISBN:0198506732